defense response to oomycetes [GO:0002229] (biological process) Regulation: regulated by regulation of defense response to oomycetes [GO:1902288]; RO_0002212 by negative regulation of defense response to oomycetes [GO:1902289]; positively regulated by GO:1902290 References: PMID:16497589 Sources: GOC:add Relationships: is a type of GO:0002239; is a type of GO:0006952 Definition: Reactions triggered in response to the presence of oomycetes that act to protect the cell or organism.